{
  "gene_name": "FYN-binding protein 2",
  "gene_symbol": "FYB2",
  "term_id": "GO:0007229",
  "gene": "UniProtKB:Q5VWT5",
  "term_label": "integrin-mediated signaling pathway"
}